{
  "gene_symbol": "RTN4",
  "gene_name": "Reticulon-4",
  "term_id": "GO:0007420",
  "term_label": "brain development",
  "gene": "UniProtKB:Q9NQC3"
}